{
  "gene_symbol": "CHD3",
  "gene": "UniProtKB:Q12873",
  "term_id": "GO:0005634",
  "term_label": "nucleus",
  "gene_name": "Chromodomain-helicase-DNA-binding protein 3"
}